{
  "term_label": "actin crosslink formation",
  "gene_symbol": "GAS2L2",
  "gene_name": "GAS2-like protein 2",
  "gene": "UniProtKB:Q8NHY3",
  "term_id": "GO:0051764"
}